{
  "term_label": "regulation of transcription by RNA polymerase II",
  "term_id": "GO:0006357",
  "gene_symbol": "ARID1A",
  "gene_name": "AT-rich interactive domain-containing protein 1A",
  "gene": "UniProtKB:O14497"
}